positive regulation of age-related resistance [GO:1904250] (biological process) Definition: Any process that activates or increases the extent of age-related resistance. References: PMID:19694953 Sources: GOC:TermGenie, GO_REF:0000058 Also known as: positive regulation of ARR, up regulation of ARR, up regulation of age-related resistance, up-regulation of ARR, up-regulation of age-related resistance, upregulation of ARR, upregulation of age-related resistance, activation of ARR, activation of adult seedling resistance, activation of age-related resistance, activation of flowering-induced resistance, activation of mature seedling resistance, activation of senescence-induced resistance, positive regulation of adult seedling resistance, positive regulation of flowering-induced resistance, positive regulation of mature seedling resistance, positive regulation of senescence-induced resistance, up regulation of adult seedling resistance, up regulation of flowering-induced resistance, up regulation of mature seedling resistance, up regulation of senescence-induced resistance, up-regulation of adult seedling resistance, up-regulation of flowering-induced resistance, up-regulation of mature seedling resistance, up-regulation of senescence-induced resistance, upregulation of adult seedling resistance, upregulation of flowering-induced resistance, upregulation of mature seedling resistance, upregulation of senescence-induced resistance Relationships: is a type of positive regulation of innate immune response [GO:0045089]; is a type of positive regulation of developmental process [GO:0051094]; is a type of regulation of age-related resistance [GO:1904248]; positively regulates GO:0090644